oncostatin-M-mediated signaling pathway [GO:0038165] (biological process) Definition: The series of molecular signals initiated by oncostatin-M (OSM) binding to its receptor on the surface of a target cell, and ending with the regulation of a downstream cellular process, e.g. transcription. OSM can signal via at least two different receptors (a specific receptor and a LIF receptor) to activate different downstream signal transduction pathways. Also known as: OSM signaling pathway, oncostatin-M signaling pathway References: PMID:10579456, PMID:12811586 Sources: GOC:nhn, GOC:signaling Relationships: is a type of cytokine-mediated signaling pathway [GO:0019221]